{
  "term_label": "nucleus",
  "gene_symbol": "SOX11",
  "term_id": "GO:0005634",
  "gene_name": "Transcription factor SOX-11",
  "gene": "UniProtKB:P35716"
}